{
  "term_label": "dolichol-phosphate-mannose synthase complex",
  "gene_symbol": "DPM2",
  "gene_name": "Dolichol phosphate-mannose biosynthesis regulatory protein",
  "term_id": "GO:0033185",
  "gene": "UniProtKB:O94777"
}